{
  "gene_symbol": "GCM1",
  "term_label": "regulation of transcription by RNA polymerase II",
  "gene": "UniProtKB:Q9NP62",
  "term_id": "GO:0006357",
  "gene_name": "Chorion-specific transcription factor GCMa"
}